{
  "gene_symbol": "TARBP2",
  "gene": "UniProtKB:Q15633",
  "term_label": "RISC-loading complex",
  "gene_name": "RISC-loading complex subunit TARBP2",
  "term_id": "GO:0070578"
}